{
  "gene_symbol": "DNAH2",
  "gene": "UniProtKB:Q9P225",
  "term_label": "axoneme",
  "term_id": "GO:0005930",
  "gene_name": "Dynein axonemal heavy chain 2"
}